{
  "term_label": "Unknown cellular component",
  "gene": "UniProtKB:Q6UW02",
  "term_id": "UNKNOWN:0003",
  "gene_symbol": "CYP20A1",
  "gene_name": "Cytochrome P450 20A1"
}